{
  "term_label": "spindle microtubule",
  "gene_symbol": "CCDC57",
  "gene": "UniProtKB:Q2TAC2",
  "term_id": "GO:0005876",
  "gene_name": "Coiled-coil domain-containing protein 57"
}